{
  "term_id": "GO:0005871",
  "gene_symbol": "KIF1A",
  "term_label": "kinesin complex",
  "gene": "UniProtKB:Q12756",
  "gene_name": "Kinesin-like protein KIF1A"
}